positive regulation of T-helper 2 cell activation [GO:2000570] (biological process) Sources: GOC:obol Relationships: is_a GO:2000516; is a type of regulation of T-helper 2 cell activation [GO:2000569]; positively regulates GO:0035712 Also known as: positive regulation of Th2 cell activation Definition: Any process that activates or increases the frequency, rate or extent of T-helper 2 cell activation.